viral capsid, turret [GO:0039670] (cellular component) References: PMID:20592081 Sources: GOC:jh2 Definition: A turret-like appendage formed at the vertices of an icosahedral capsid. Relationships: is a type of viral capsid, decoration [GO:0098021]; BFO_0000050 icosahedral viral capsid [GO:0019030]